{
  "gene_symbol": "IRS1",
  "term_label": "phosphatidylinositol 3-kinase binding",
  "gene": "UniProtKB:P35568",
  "gene_name": "Insulin receptor substrate 1",
  "term_id": "GO:0043548"
}